naringenin 2-hydroxylase activity [GO:0102469] (molecular function) Relationships: is a type of oxidoreductase activity, acting on paired donors, with incorporation or reduction of molecular oxygen, reduced flavin or flavoprotein as one donor, and incorporation of one atom of oxygen [GO:0016712] Definition: Catalysis of the reaction:(2S)-naringenin + O2 + reduced [NADPH--hemoprotein reductase] = (2S)-2-hydroxynaringenin + H(+) + H2O + oxidized [NADPH--hemoprotein reductase]. Sources: RHEA:57588